{
  "gene_symbol": "ZNF365",
  "term_label": "regulation of neuron projection development",
  "gene": "UniProtKB:Q70YC5",
  "term_id": "GO:0010975",
  "gene_name": "Protein ZNF365"
}